{
  "gene": "UniProtKB:Q8N4S7",
  "gene_symbol": "PAQR4",
  "term_id": "UNKNOWN:0002",
  "term_label": "Unknown biological process",
  "gene_name": "Progestin and adipoQ receptor family member 4"
}